ethylene receptor activity [GO:0038199] (molecular function) Also known as: C2H4 receptor activity, ethylene response sensor References: PMID:22467798, PMID:24012247 Sources: GOC:signaling Definition: Combining with ethylene and transmitting the signal in the cell to initiate a change in cell activity. Relationships: is a type of signaling receptor activity [GO:0038023]; is part of ethylene-activated signaling pathway [GO:0009873]; has part GO:0051740 Subtypes: ethylene receptor histidine kinase activity [GO:0038200]